hemopoiesis [GO:0030097] (biological process) Sources: GOC:dgh, ISBN:0198506732 Definition: The process whose specific outcome is the progression of the myeloid and lymphoid derived organ/tissue systems of the blood and other parts of the body over time, from formation to the mature structure. The site of hemopoiesis is variable during development, but occurs primarily in bone marrow or kidney in many adult vertebrates. Also known as: blood cell biosynthesis, blood cell formation, haemopoiesis, hematopoiesis Regulation: regulated by regulation of hemopoiesis [GO:1903706]; negatively regulated by negative regulation of hemopoiesis [GO:1903707]; RO_0002213 by positive regulation of hemopoiesis [GO:1903708] Relationships: is a type of cell development [GO:0048468] Subtypes: hemocyte development [GO:0007516], embryonic hemopoiesis [GO:0035162], post-embryonic hemopoiesis [GO:0035166], definitive hemopoiesis [GO:0060216], myeloid cell development [GO:0061515]